{
  "term_id": "UNKNOWN:0002",
  "gene_name": "Protein RD3-like",
  "gene_symbol": "RD3L",
  "gene": "UniProtKB:P0DJH9",
  "term_label": "Unknown biological process"
}